{
  "term_id": "GO:0019369",
  "gene_name": "Polyunsaturated fatty acid lipoxygenase ALOX15",
  "term_label": "arachidonate metabolic process",
  "gene_symbol": "ALOX15",
  "gene": "UniProtKB:P16050"
}